negative regulation of non-canonical Wnt signaling pathway [GO:2000051] (biological process) Sources: GOC:obol, GOC:yaf Also known as: negative regulation of beta-catenin-independent Wnt receptor signaling pathway, negative regulation of non-canonical Wnt receptor signaling pathway, negative regulation of non-canonical Wnt receptor signalling pathway, negative regulation of non-canonical Wnt-activated signaling pathway Subtypes: negative regulation of Wnt signaling pathway, calcium modulating pathway [GO:0045812], GO:0140712, negative regulation of Wnt signaling pathway, planar cell polarity pathway [GO:0141113] Relationships: is a type of negative regulation of Wnt signaling pathway [GO:0030178]; is a type of regulation of non-canonical Wnt signaling pathway [GO:2000050]; negatively regulates non-canonical Wnt signaling pathway [GO:0035567] Definition: Any process that stops, prevents, or reduces the frequency, rate or extent of non-canonical Wnt signaling pathway.